{
  "term_id": "GO:0000086",
  "gene_symbol": "CDK4",
  "term_label": "G2/M transition of mitotic cell cycle",
  "gene": "UniProtKB:P11802",
  "gene_name": "Cyclin-dependent kinase 4"
}